{
  "term_id": "GO:0006511",
  "gene": "UniProtKB:P53804",
  "gene_symbol": "TTC3",
  "gene_name": "E3 ubiquitin-protein ligase TTC3",
  "term_label": "ubiquitin-dependent protein catabolic process"
}